2-hydroxy-6-oxo-6-(2'-aminophenyl)hexa-2,4-dienoate hydrolase activity [GO:0018768] (molecular function) Definition: Catalysis of the reaction: (2E,4E)-6-(2-aminophenyl)-2-hydroxy-6-oxohexa-2,4-dienoate + H2O = (2E)-2-hydroxypenta-2,4-dienoate + anthranilate + H+. Relationships: is a type of hydrolase activity, acting on acid carbon-carbon bonds, in ketonic substances [GO:0016823] Sources: RHEA:27870